{
  "term_id": "GO:0046969",
  "gene_symbol": "SIRT1",
  "gene_name": "NAD-dependent protein deacetylase sirtuin-1",
  "gene": "UniProtKB:Q96EB6",
  "term_label": "histone H3K9 deacetylase activity, NAD-dependent"
}